cobalt-factor II C20-methyltransferase activity [GO:0043781] (molecular function) Relationships: is a type of methyltransferase activity [GO:0008168] Definition: Catalysis of the reaction: S-adenosyl-L-methionine + cobalt-factor II = S-adenosyl-L-homocysteine + cobalt-factor III. Also known as: cobalt-factor II C20 methyltransferase activity, CbiL, S-adenosyl-L-methionine:cobalt-factor-II C20-methyltransferase activity, cobalt-precorrin-2 C(20)-methyltransferase activity Sources: EC:2.1.1.151